{
  "gene_symbol": "GRXCR2",
  "term_id": "GO:0120043",
  "term_label": "stereocilium shaft",
  "gene_name": "Glutaredoxin domain-containing cysteine-rich protein 2",
  "gene": "UniProtKB:A6NFK2"
}